{
  "term_label": "regulation of canonical Wnt signaling pathway",
  "term_id": "GO:0060828",
  "gene": "UniProtKB:Q8N944",
  "gene_name": "APC membrane recruitment protein 3",
  "gene_symbol": "AMER3"
}